negative regulation of response to endoplasmic reticulum stress [GO:1903573] (biological process) Definition: Any process that stops, prevents or reduces the frequency, rate or extent of a response to endoplasmic reticulum stress. References: PMID:11381086 Sources: GOC:PARL, GOC:TermGenie, GOC:bf, GO_REF:0000058 Relationships: is a type of negative regulation of cellular process [GO:0048523]; is a type of GO:0048585; is a type of GO:1905897; negatively regulates GO:0034976 Subtypes: negative regulation of endoplasmic reticulum unfolded protein response [GO:1900102], negative regulation of endoplasmic reticulum stress-induced intrinsic apoptotic signaling pathway [GO:1902236], negative regulation of ERAD pathway [GO:1904293] Also known as: down regulation of ER stress response, down regulation of cellular response to endoplasmic reticulum stress, down regulation of response to ER stress, down regulation of response to endoplasmic reticulum stress, down-regulation of ER stress response, down-regulation of cellular response to endoplasmic reticulum stress, down-regulation of response to ER stress, down-regulation of response to endoplasmic reticulum stress, downregulation of ER stress response, downregulation of cellular response to endoplasmic reticulum stress, downregulation of response to ER stress, downregulation of response to endoplasmic reticulum stress, negative regulation of ER stress response, negative regulation of cellular response to endoplasmic reticulum stress, negative regulation of response to ER stress, inhibition of ER stress response, inhibition of cellular response to endoplasmic reticulum stress, inhibition of response to ER stress, inhibition of response to endoplasmic reticulum stress